{
  "gene_symbol": "CDC5L",
  "gene": "UniProtKB:Q99459",
  "gene_name": "Cell division cycle 5-like protein",
  "term_id": "GO:0000977",
  "term_label": "RNA polymerase II transcription regulatory region sequence-specific DNA binding"
}